{
  "term_label": "synaptic vesicle",
  "gene": "UniProtKB:Q12829",
  "gene_symbol": "RAB40B",
  "gene_name": "Ras-related protein Rab-40B",
  "term_id": "GO:0008021"
}